{
  "term_label": "rRNA processing",
  "gene_symbol": "DDX10",
  "term_id": "GO:0006364",
  "gene": "UniProtKB:Q13206",
  "gene_name": "Probable ATP-dependent RNA helicase DDX10"
}